{
  "gene_symbol": "TOR3A",
  "term_label": "Unknown biological process",
  "term_id": "UNKNOWN:0002",
  "gene": "UniProtKB:Q9H497",
  "gene_name": "Torsin-3A"
}